L-serine biosynthetic process [GO:0006564] (biological process) Definition: The chemical reactions and pathways resulting in the formation of L-serine, the L-enantiomer of serine, i.e. (2S)-2-amino-3-hydroxypropanoic acid. Sources: GOC:ai, GOC:jsg Also known as: L-serine anabolism, L-serine biosynthesis, L-serine formation, L-serine synthesis Relationships: is a type of L-serine metabolic process [GO:0006563]; is a type of serine family amino acid biosynthetic process [GO:0009070]; is a type of L-amino acid biosynthetic process [GO:0170034]; is a type of proteinogenic amino acid biosynthetic process [GO:0170038]